{
  "gene_name": "Brain-specific angiogenesis inhibitor 1-associated protein 2",
  "gene_symbol": "BAIAP2",
  "term_label": "nucleoplasm",
  "term_id": "GO:0005654",
  "gene": "UniProtKB:Q9UQB8"
}